{
  "term_label": "Unknown molecular function",
  "gene_name": "Pleckstrin homology domain-containing family G member 6",
  "gene_symbol": "PLEKHG6",
  "gene": "UniProtKB:Q3KR16",
  "term_id": "UNKNOWN:0001"
}